{
  "term_id": "GO:0004062",
  "gene": "UniProtKB:Q6IMI6",
  "gene_name": "Sulfotransferase 1C3",
  "term_label": "aryl sulfotransferase activity",
  "gene_symbol": "SULT1C3"
}